lysophosphatidylserine flippase activity [GO:0180013] (molecular function) Definition: Catalysis of the movement of a lysophosphatidylserine from the exoplasmic to the cytosolic leaflet of a membrane, using energy from the hydrolysis of ATP. References: PMID:34645814 Relationships: is a type of glycerophospholipid flippase activity [GO:0140333]